{
  "gene": "UniProtKB:P10155",
  "gene_symbol": "RO60",
  "gene_name": "RNA-binding protein RO60",
  "term_label": "Unknown biological process",
  "term_id": "UNKNOWN:0002"
}